positive regulation of synapse pruning [GO:1905808] (biological process) Definition: Any process that activates or increases the frequency, rate or extent of synapse pruning. References: PMID:27779093 Sources: GOC:TermGenie, GO_REF:0000058 Relationships: is a type of positive regulation of cellular component organization [GO:0051130]; is a type of regulation of synapse pruning [GO:1905806]; positively regulates synapse pruning [GO:0098883] Also known as: regulation of synapse clearance, regulation of synapse disassembly, regulation of synapse elimination, regulation of synapse removal, up regulation of synapse disassembly, up-regulation of synapse disassembly, upregulation of synapse disassembly, activation of synapse disassembly